{
  "term_label": "Unknown molecular function",
  "gene_symbol": "Q8N976",
  "gene_name": "Putative uncharacterized protein FLJ38264",
  "term_id": "UNKNOWN:0001",
  "gene": "UniProtKB:Q8N976"
}